{
  "term_label": "positive regulation of transcription by RNA polymerase II",
  "gene": "UniProtKB:Q15699",
  "gene_name": "ALX homeobox protein 1",
  "gene_symbol": "ALX1",
  "term_id": "GO:0045944"
}